{
  "gene": "UniProtKB:Q6PIU1",
  "gene_name": "Potassium voltage-gated channel subfamily V member 1",
  "term_id": "GO:0016020",
  "gene_symbol": "KCNV1",
  "term_label": "membrane"
}